{
  "gene_name": "Dynamin-2",
  "gene": "UniProtKB:P50570",
  "term_id": "GO:0031623",
  "term_label": "receptor internalization",
  "gene_symbol": "DNM2"
}